keratan sulfate proteoglycan catabolic process [GO:0042340] (biological process) Also known as: keratan sulfate breakdown, keratan sulfate catabolism, keratan sulfate degradation, keratan sulphate catabolic process, keratan sulphate catabolism Relationships: is a type of GO:0030167; is a type of keratan sulfate proteoglycan metabolic process [GO:0042339] References: PMID:35536982 Definition: The chemical reactions and pathways resulting in the breakdown of keratan sulfate proteoglycans, which consist of a core protein linked to a keratan sulfate glycosaminoglycan. The keratan sulfate chain is composed of the repeating disaccharide unit beta-(1,4)-N-acetyl-D-glucosamine-beta-(1,3)-galactose, both of which can be sulfated.